chemorepulsion involved in interneuron migration from the subpallium to the cortex [GO:0021842] (biological process) References: PMID:12626695 Sources: GOC:cls, GOC:dgh, GOC:dph, GOC:jid, GO_REF:0000021 Also known as: negative chemotaxis involved in interneuron migration from the subpallium to the cortex Definition: The creation and reception of signals that result in the movement of interneurons away from the signal during migration from the subpallium to the cortex. Relationships: is a type of negative chemotaxis [GO:0050919]; is part of GO:0021840